positive regulation of hemocyte differentiation [GO:0045612] (biological process) Definition: Any process that activates or increases the frequency, rate or extent of hemocyte differentiation. Also known as: positive regulation of arthropod blood cell differentiation, up regulation of hemocyte differentiation, up-regulation of hemocyte differentiation, upregulation of hemocyte differentiation, activation of hemocyte differentiation, stimulation of hemocyte differentiation Subtypes: GO:0035205, positive regulation of crystal cell differentiation [GO:0042691], positive regulation of plasmatocyte differentiation [GO:0045615] Relationships: is a type of positive regulation of immune system process [GO:0002684]; is a type of GO:0045597; is a type of GO:0045610; positively regulates hemocyte differentiation [GO:0042386] Sources: GOC:go_curators